{
  "gene_name": "B2 bradykinin receptor",
  "gene": "UniProtKB:P30411",
  "gene_symbol": "BDKRB2",
  "term_id": "GO:0042311",
  "term_label": "vasodilation"
}